{
  "gene_symbol": "PRKACB",
  "term_label": "adenylate cyclase-activating G protein-coupled receptor signaling pathway",
  "gene": "UniProtKB:P22694",
  "gene_name": "cAMP-dependent protein kinase catalytic subunit beta",
  "term_id": "GO:0007189"
}